{
  "gene_name": "Protein moonraker",
  "gene": "UniProtKB:Q2KHM9",
  "term_label": "protein localization to centrosome",
  "term_id": "GO:0071539",
  "gene_symbol": "KIAA0753"
}